{
  "term_label": "Golgi apparatus",
  "gene_symbol": "ZDHHC22",
  "term_id": "GO:0005794",
  "gene_name": "Palmitoyltransferase ZDHHC22",
  "gene": "UniProtKB:Q8N966"
}